noradrenergic neuron differentiation [GO:0003357] (biological process) Relationships: is a type of neuron differentiation [GO:0030182] Subtypes: GO:0003361 Also known as: norepinephrine secreting neuron differentiation Sources: GOC:dph Definition: The process in which a relatively unspecialized cell acquires specialized features of an noradrenergic neuron, a neuron that secretes noradrenaline.